{
  "gene": "UniProtKB:Q8WXS4",
  "term_label": "Unknown cellular component",
  "term_id": "UNKNOWN:0003",
  "gene_name": "Voltage-dependent calcium channel gamma-like subunit",
  "gene_symbol": "TMEM37"
}